{
  "term_id": "GO:0003729",
  "gene": "UniProtKB:Q9BYJ9",
  "term_label": "mRNA binding",
  "gene_symbol": "YTHDF1",
  "gene_name": "YTH domain-containing family protein 1"
}